{
  "gene_name": "Ras GTPase-activating protein-binding protein 2",
  "gene_symbol": "G3BP2",
  "term_id": "GO:0034063",
  "term_label": "stress granule assembly",
  "gene": "UniProtKB:Q9UN86"
}